acetate kinase activity [GO:0008776] (MF) Definition: Catalysis of the reaction: ATP + acetate = ADP + acetyl phosphate. Sources: EC:2.7.2.1 Also known as: AK activity, ATP:acetate phosphotransferase activity, AckA, acetate kinase (phosphorylating) activity, acetic kinase activity, acetokinase activity Relationships: is a type of kinase activity [GO:0016301]; is a type of phosphotransferase activity, carboxyl group as acceptor [GO:0016774]